{
  "gene": "UniProtKB:Q96AJ1",
  "gene_name": "Clusterin-associated protein 1",
  "term_label": "microtubule organizing center",
  "gene_symbol": "CLUAP1",
  "term_id": "GO:0005815"
}